{
  "term_label": "negative regulation of cytoplasmic translation",
  "gene": "UniProtKB:Q9BZB8",
  "gene_symbol": "CPEB1",
  "gene_name": "Cytoplasmic polyadenylation element-binding protein 1",
  "term_id": "GO:2000766"
}